response to polyamine macromolecule [GO:1904583] (biological process) Also known as: response to polyamine, response to polyamines Subtypes: cellular response to polyamine macromolecule [GO:1904584] References: PMID:20805360 Sources: GOC:TermGenie, GO_REF:0000071 Definition: Any process that results in a change in state or activity of a cell or an organism (in terms of movement, secretion, enzyme production, gene expression, etc.) as a result of a polyamine macromolecule stimulus. Relationships: is a type of response to nitrogen compound [GO:1901698]